{
  "gene_name": "Angiomotin-like protein 1",
  "gene": "UniProtKB:Q8IY63",
  "term_id": "GO:0031410",
  "term_label": "cytoplasmic vesicle",
  "gene_symbol": "AMOTL1"
}